cellular response to decreased oxygen levels [GO:0036294] (biological process) Sources: GOC:al Subtypes: cellular response to anoxia [GO:0071454], cellular response to hypoxia [GO:0071456], cellular response to oxygen-glucose deprivation [GO:0090650] Note: This term should be used when a decrease in oxygen levels is not considered a stress response. For a hypoxic stress response, consider instead 'cellular response to hypoxia ; GO:0071456'. Also known as: cellular response to lowered oxygen levels Relationships: is a type of response to decreased oxygen levels [GO:0036293]; is a type of cellular response to oxygen levels [GO:0071453] Definition: Any process that results in a change in state or activity of a cell (in terms of movement, secretion, enzyme production, gene expression, etc.) as a result of a stimulus reflecting a decline in the level of oxygen.